acrolein reductase activity [GO:0102232] (molecular function) Definition: Catalysis of the reaction: acrolein + NADPH + H+ = propanal + NADP. Relationships: is a type of GO:0016628 References: PMID:21169366 Sources: GOC:pz